substrate adhesion-dependent cell spreading [GO:0034446] (biological process) Relationships: is a type of cell-substrate adhesion [GO:0031589] Regulation: regulated by regulation of substrate adhesion-dependent cell spreading [GO:1900024]; negatively regulated by GO:1900025; positively regulated by positive regulation of substrate adhesion-dependent cell spreading [GO:1900026] References: PMID:17050732 Sources: GOC:mah, GOC:pf Definition: The morphogenetic process that results in flattening of a cell as a consequence of its adhesion to a substrate. Also known as: cell spreading during cell substrate adhesion, substrate adhesion dependent cell spreading